{
  "term_id": "GO:0005783",
  "gene_name": "Protein canopy homolog 2",
  "gene": "UniProtKB:Q9Y2B0",
  "term_label": "endoplasmic reticulum",
  "gene_symbol": "CNPY2"
}